{
  "gene_name": "Pre-mRNA cleavage complex 2 protein Pcf11",
  "gene_symbol": "PCF11",
  "gene": "UniProtKB:O94913",
  "term_label": "mRNA cleavage factor complex",
  "term_id": "GO:0005849"
}